alae of collagen and cuticulin-based cuticle extracellular matrix [GO:0060111] (cellular component) Definition: Raised, thickened cuticular ridges that run longitudinally, and in parallel, along the left and right sides of the animal. The alae lie above the hypodermal cells known as the lateral seam cells. In C. elegans, alae are produced in L1 larvae, dauer larvae and adult stage animals, where they consist of three, five, and three ridges of distinct morphology, respectively. Also known as: alae of collagen and cuticulin-based exoskeleton extracellular matrix Sources: GOC:dph, GOC:kmv, ISSN:15518507 Relationships: is_a cellular anatomical structure [GO:0110165]; is part of cuticular extracellular matrix [GO:0060102]